microglial cell proliferation [GO:0061518] (biological process) References: PMID:17344397 Sources: GOC:dph Definition: The expansion of a microglial cell population by cell division. Relationships: is a type of glial cell proliferation [GO:0014009]; is a type of macrophage proliferation [GO:0061517]